{
  "gene_symbol": "ZNF675",
  "term_id": "GO:0006355",
  "gene": "UniProtKB:Q8TD23",
  "gene_name": "Zinc finger protein 675",
  "term_label": "regulation of DNA-templated transcription"
}